{
  "gene_symbol": "PI4KB",
  "term_label": "phosphatidylinositol phosphate biosynthetic process",
  "gene_name": "Phosphatidylinositol 4-kinase beta",
  "term_id": "GO:0046854",
  "gene": "UniProtKB:Q9UBF8"
}